lamellipodium organization [GO:0097581] (biological process) Subtypes: lamellipodium assembly [GO:0030032], lamellipodium morphogenesis [GO:0072673] Relationships: is a type of GO:0120036 Regulation: regulated by regulation of lamellipodium organization [GO:1902743]; negatively regulated by GO:1902744; positively regulated by GO:1902745 References: PMID:16054028 Sources: GOC:als Definition: A process that is carried out at the cellular level which results in the assembly, arrangement of constituent parts, or disassembly of a lamellipodium. A lamellipodium is a thin sheetlike process extended by the leading edge of a crawling fibroblast; contains a dense meshwork of actin filaments.